Schaffer axon collateral [GO:1990021] (cellular component) Relationships: is a type of GO:0044303 Sources: NIF_Subcellular:nlx_subcell_20090511 Definition: Part of axon of a CA3 pyramidal neuron that projects to hippocampal area CA1. Also known as: Schaffer collateral